{
  "gene_name": "Electron transfer flavoprotein regulatory factor 1",
  "gene_symbol": "ETFRF1",
  "term_id": "UNKNOWN:0001",
  "gene": "UniProtKB:Q6IPR1",
  "term_label": "Unknown molecular function"
}